{
  "gene": "UniProtKB:Q05516",
  "gene_symbol": "ZBTB16",
  "gene_name": "Zinc finger and BTB domain-containing protein 16",
  "term_label": "regulation of transcription by RNA polymerase II",
  "term_id": "GO:0006357"
}